dopamine transport [GO:0015872] (biological process) Subtypes: dopamine secretion [GO:0014046], dopamine uptake [GO:0090494] Relationships: is a type of catecholamine transport [GO:0051937] Sources: GOC:ai Definition: The directed movement of dopamine into, out of or within a cell, or between cells, by means of some agent such as a transporter or pore. Dopamine is a catecholamine neurotransmitter and a metabolic precursor of noradrenaline and adrenaline.